somatic diversification of T cell receptor genes [GO:0002568] (BP) Also known as: somatic diversification of TCR genes Relationships: is_a somatic diversification of immune receptors [GO:0002200]; BFO_0000050 GO:0030217 Definition: The somatic process that results in the generation of sequence diversity of T cell receptor genes. Sources: GOC:add, ISBN:0781735149 Subtypes: somatic diversification of T cell receptor genes by N region addition [GO:0002571], somatic recombination of T cell receptor gene segments [GO:0002681]